{
  "term_label": "structural constituent of skin epidermis",
  "gene_symbol": "KRT72",
  "term_id": "GO:0030280",
  "gene_name": "Keratin, type II cytoskeletal 72",
  "gene": "UniProtKB:Q14CN4"
}